{
  "term_label": "cytokine activity",
  "gene_symbol": "GDF6",
  "term_id": "GO:0005125",
  "gene": "UniProtKB:Q6KF10",
  "gene_name": "Growth_differentiation factor 6"
}